{
  "gene": "UniProtKB:P41247",
  "term_id": "GO:0005811",
  "term_label": "lipid droplet",
  "gene_symbol": "PNPLA4",
  "gene_name": "Patatin-like phospholipase domain-containing protein 4"
}